ABC-type sterol transporter activity [GO:0034041] (molecular function) Definition: Enables the transfer of a solute or solutes from one side of a membrane to the other according to the reaction: ATP + H2O + sterol(in) = ADP + phosphate + sterol(out). Sources: GOC:BHF, GOC:rl Also known as: ATP-coupled sterol transmembrane transporter activity, ATP-dependent sterol transmembrane transporter activity, ATPase-coupled sterol transmembrane transporter activity, sterol-transporting ATPase activity Relationships: is a type of ATPase-coupled lipid transmembrane transporter activity [GO:0034040]; is a type of ABC-type transporter activity [GO:0140359]